{
  "gene": "UniProtKB:Q15465",
  "gene_name": "Sonic hedgehog protein",
  "term_id": "GO:0005509",
  "term_label": "calcium ion binding",
  "gene_symbol": "SHH"
}